meristem growth [GO:0035266] (biological process) Definition: The increase in size or mass of a meristem, a region of tissue in a plant that is composed of one or more undifferentiated cells capable of undergoing mitosis and differentiation. Regulation: regulated by regulation of meristem growth [GO:0010075] Subtypes: vegetative meristem growth [GO:0010448], root meristem growth [GO:0010449], inflorescence meristem growth [GO:0010450], GO:0010451 Relationships: is a type of developmental growth [GO:0048589]; is part of meristem development [GO:0048507] Sources: GOC:bf, ISBN:0198547684